{
  "gene": "UniProtKB:A4QN01",
  "gene_symbol": "LINC01553",
  "term_label": "Unknown molecular function",
  "term_id": "UNKNOWN:0001",
  "gene_name": "Putative uncharacterized protein encoded by LINC01553"
}